{
  "term_id": "GO:0008643",
  "gene": "UniProtKB:Q9BRV3",
  "gene_symbol": "SLC50A1",
  "gene_name": "Sugar transporter SWEET1",
  "term_label": "carbohydrate transport"
}